regulation of renin secretion into blood stream [GO:1900133] (BP) Subtypes: GO:1900134, positive regulation of renin secretion into blood stream [GO:1900135] Also known as: regulation of renin release into blood stream Sources: GOC:TermGenie Definition: Any process that modulates the frequency, rate or extent of renin secretion into blood stream. Relationships: is a type of regulation of systemic arterial blood pressure [GO:0003073]; is a type of regulation of endocrine process [GO:0044060]; is a type of GO:0050708; is a type of regulation of renal system process [GO:0098801]; regulates renin secretion into blood stream [GO:0002001]